{
  "term_id": "GO:0050839",
  "gene": "UniProtKB:Q9UN67",
  "gene_name": "Protocadherin beta-10",
  "gene_symbol": "PCDHB10",
  "term_label": "cell adhesion molecule binding"
}